negative regulation of constitutive secretory pathway [GO:1903434] (biological process) Definition: Any process that stops, prevents or reduces the frequency, rate or extent of constitutive secretory pathway. Relationships: is a type of negative regulation of exocytosis [GO:0045920]; is a type of regulation of constitutive secretory pathway [GO:1903433]; negatively regulates constitutive secretory pathway [GO:0045054] Also known as: down regulation of constitutive secretory pathway, down-regulation of constitutive secretory pathway, downregulation of constitutive secretory pathway, inhibition of constitutive secretory pathway References: PMID:22899725 Sources: GOC:TermGenie, GOC:als, GO_REF:0000058